{
  "gene_name": "Zinc finger protein 567",
  "gene": "UniProtKB:Q8N184",
  "term_id": "GO:0000978",
  "gene_symbol": "ZNF567",
  "term_label": "RNA polymerase II cis-regulatory region sequence-specific DNA binding"
}